corticotropin-releasing hormone receptor activity [GO:0043404] (molecular function) Definition: Combining with corticotropin-releasing hormone and transmitting the signal to initiate a change in cell activity. References: PMID:11027914, PMID:15134857 Sources: GOC:signaling, ISBN:0838577016 Also known as: CRF receptor activity, CRH receptor activity, adrenocorticotropin-releasing hormone receptor activity, corticotropin-releasing factor receptor activity Relationships: is a type of GO:0038023; is part of hormone-mediated signaling pathway [GO:0009755]; has part corticotropin-releasing hormone binding [GO:0051424] Regulation: negatively regulated by negative regulation of corticotropin-releasing hormone receptor activity [GO:1900011]